{
  "term_label": "immunoglobulin mediated immune response",
  "term_id": "GO:0016064",
  "gene_symbol": "IGHV2-26",
  "gene": "UniProtKB:A0A0B4J1V2",
  "gene_name": "Immunoglobulin heavy variable 2-26"
}